chromoplast [GO:0009509] (CC) Relationships: is a type of GO:0009536 Sources: ISBN:0471245208 Definition: A plastid containing pigments other than chlorophyll, usually yellow and orange carotenoid pigments.